{
  "gene_name": "Putative U2 small nuclear ribonucleoprotein auxiliary factor 35 kDa subunit-related protein 1",
  "term_label": "spliceosomal complex",
  "gene": "UniProtKB:Q15695",
  "term_id": "GO:0005681",
  "gene_symbol": "ZRSR2P1"
}